{
  "gene": "UniProtKB:Q96A59",
  "gene_name": "MARVEL domain-containing protein 3",
  "term_label": "Unknown molecular function",
  "gene_symbol": "MARVELD3",
  "term_id": "UNKNOWN:0001"
}